oocyte nucleus localization involved in oocyte dorsal/ventral axis specification [GO:0051663] (biological process) Sources: GOC:ai, GOC:dph, GOC:mtg_sensu, GOC:tb Subtypes: oocyte nucleus migration involved in oocyte dorsal/ventral axis specification [GO:0007312], maintenance of oocyte nucleus location involved in oocyte dorsal/ventral axis specification [GO:0042070] Definition: The directed movement of the nucleus to a specific location within a cell during the establishment and maintenance of the dorsal/ventral axis of the oocyte. Relationships: is a type of GO:0051647; is part of oocyte dorsal/ventral axis specification [GO:0007310] Also known as: establishment and maintenance of oocyte nucleus localization during oocyte axis determination, oocyte axis determination, oocyte nucleus localization, oocyte nucleus localisation involved in oocyte dorsal/ventral axis specification, oocyte nucleus localization involved in oocyte dorsal-ventral axis specification, oocyte nucleus localization involved in oocyte dorsal/ventral axis determination, oocyte nucleus localization involved in oocyte dorsoventral axis specification, oocyte nucleus localization during oocyte axis determination